{
  "gene_symbol": "ADGRA1",
  "gene_name": "Adhesion G protein-coupled receptor A1",
  "term_id": "UNKNOWN:0001",
  "term_label": "Unknown molecular function",
  "gene": "UniProtKB:Q86SQ6"
}